{
  "gene_symbol": "CIITA",
  "gene": "UniProtKB:P33076",
  "term_label": "positive regulation of transcription by RNA polymerase II",
  "term_id": "GO:0045944",
  "gene_name": "MHC class II transactivator"
}